{
  "term_id": "GO:0000978",
  "gene": "UniProtKB:Q9HCS4",
  "gene_symbol": "TCF7L1",
  "term_label": "RNA polymerase II cis-regulatory region sequence-specific DNA binding",
  "gene_name": "Transcription factor 7-like 1"
}